{
  "term_id": "GO:0030515",
  "gene_name": "WD repeat-containing protein 3",
  "term_label": "snoRNA binding",
  "gene": "UniProtKB:Q9UNX4",
  "gene_symbol": "WDR3"
}